glycerol dehydratase activity [GO:0046405] (molecular function) References: PMID:18307109 Sources: EC:4.2.1.30 Also known as: glycerol dehydrase activity, glycerol hydro-lyase (3-hydroxypropanal-forming), glycerol hydro-lyase activity Relationships: is_a hydro-lyase activity [GO:0016836] Definition: Catalysis of the reaction: glycerol = 3-hydroxypropanal + H2O.